{
  "term_label": "actin cytoskeleton",
  "gene_name": "Beta-actin-like protein 2",
  "gene_symbol": "ACTBL2",
  "gene": "UniProtKB:Q562R1",
  "term_id": "GO:0015629"
}